{
  "term_id": "UNKNOWN:0002",
  "gene_symbol": "SH3BGRL2",
  "gene_name": "SH3 domain-binding glutamic acid-rich-like protein 2",
  "term_label": "Unknown biological process",
  "gene": "UniProtKB:Q9UJC5"
}